urothelial cell proliferation [GO:0050674] (biological process) Definition: The multiplication or reproduction of urothelial cells, resulting in the expansion of a cell population. Urothelial cells make up a layer of transitional epithelium in the wall of the bladder, ureter, and renal pelvis, external to the lamina propria. Sources: ISBN:0721662544 Relationships: is a type of epithelial cell proliferation [GO:0050673] Regulation: regulated by GO:0050675; negatively regulated by negative regulation of urothelial cell proliferation [GO:0050676]; positively regulated by positive regulation of urothelial cell proliferation [GO:0050677]